positive regulation of MAPKKK cascade by fibroblast growth factor receptor signaling pathway [GO:0090080] (biological process) Definition: The series of molecular signals generated as a consequence of a fibroblast growth factor receptor binding to one of its physiological ligands resulting in an increase in the rate or frequency of a MAPKKK cascade. Sources: GOC:dph, GOC:tb Also known as: positive regulation of MAPKKK cascade by fibroblast growth factor receptor signalling pathway Relationships: is_a fibroblast growth factor receptor signaling pathway [GO:0008543]; is a type of positive regulation of MAPK cascade [GO:0043410]